{
  "gene_name": "Serine_threonine-protein kinase PAK 3",
  "gene_symbol": "PAK3",
  "term_id": "GO:0004674",
  "gene": "UniProtKB:O75914",
  "term_label": "protein serine/threonine kinase activity"
}